{
  "gene": "UniProtKB:Q9H0V1",
  "gene_name": "Transmembrane protein 168",
  "term_label": "Unknown molecular function",
  "gene_symbol": "TMEM168",
  "term_id": "UNKNOWN:0001"
}